{
  "gene_symbol": "ARHGDIB",
  "term_id": "GO:0007266",
  "term_label": "Rho protein signal transduction",
  "gene": "UniProtKB:P52566",
  "gene_name": "Rho GDP-dissociation inhibitor 2"
}